scytalone dehydratase activity [GO:0030411] (molecular function) Also known as: scytalone 7,8-hydro-lyase (1,3,8-trihydroxynaphthalene-forming), scytalone 7,8-hydro-lyase activity Definition: Catalysis of the reaction: scytalone = 1,3,8-trihydroxynaphthalene + H2O. Sources: EC:4.2.1.94, RHEA:24396 Relationships: is a type of hydro-lyase activity [GO:0016836]